{
  "term_label": "vesicle-mediated transport",
  "term_id": "GO:0016192",
  "gene_name": "Synaptotagmin-12",
  "gene_symbol": "SYT12",
  "gene": "UniProtKB:Q8IV01"
}